DNA-templated viral transcription [GO:0039695] (biological process) Sources: GOC:bf, GOC:jl Relationships: is a type of viral transcription [GO:0019083] Definition: A transcription process that uses a viral DNA as a template.